procyclogenesis [GO:0120324] (BP) Definition: The morphological, biochemical and genetic changes that induce the differentiation of bloodstream form trypomastigotes into procyclic trypomastigotes in some of the Trypanosomatidae species such as Trypanosoma brucei. This process occurs inside the midgut of the tsetse fly vectors in T. brucei. Relationships: is a type of development of symbiont in host [GO:0044114] References: PMID:10593184, PMID:1698624, PMID:17997129, PMID:3194362, PMID:3194363 Sources: GOC:ach